myelin assembly [GO:0032288] (biological process) Subtypes: central nervous system myelin formation [GO:0032289], GO:0032290 Definition: The process in which the wraps of cell membrane that constitute myelin are laid down around an axon in the central or peripheral nervous system. Also known as: myelin sheath assembly, myelin formation Sources: GOC:dgh, GOC:dph, GOC:tb Relationships: is a type of cellular component assembly involved in morphogenesis [GO:0010927]; is part of myelination [GO:0042552]